{
  "gene_symbol": "TMEM88",
  "gene_name": "Transmembrane protein 88",
  "term_label": "negative regulation of canonical Wnt signaling pathway",
  "gene": "UniProtKB:Q6PEY1",
  "term_id": "GO:0090090"
}